MCM complex [GO:0042555] (cellular component) Definition: A hexameric protein complex required for the initiation and regulation of DNA replication. References: PMID:11282021 Sources: GOC:jl Relationships: is a type of GO:0032991; has part MCM core complex [GO:0097373] Also known as: mini-chromosome maintenance complex Subtypes: GO:0097362